{
  "term_id": "GO:0009311",
  "gene_name": "Alpha-N-acetylgalactosaminide alpha-2,6-sialyltransferase 3",
  "term_label": "oligosaccharide metabolic process",
  "gene": "UniProtKB:Q8NDV1",
  "gene_symbol": "ST6GALNAC3"
}